{
  "gene_name": "Cardiotrophin-1",
  "term_label": "cell surface receptor signaling pathway via JAK-STAT",
  "gene_symbol": "CTF1",
  "gene": "UniProtKB:Q16619",
  "term_id": "GO:0007259"
}